phagolysosome vesicle membrane [GO:0106175] (cellular component) Relationships: is a type of cytoplasmic vesicle membrane [GO:0030659]; is part of phagolysosome [GO:0032010] References: PMID:29471269 Sources: GOC:pde Definition: The lipid bylayer surrounding a phagolysosome.